response to 5-fluorouracil [GO:0036275] (biological process) Definition: Any process that results in a change in state or activity of a cell or an organism (in terms of movement, secretion, enzyme production, gene expression, etc.) as a result of a 5-fluorouracil stimulus. Relationships: is a type of response to chemical [GO:0042221] Sources: GOC:hp Also known as: response to 5-fluoropyrimidine-2,4(1H,3H)-dione, response to fluorouracil Note: Note that this term is in the subset of terms that should not be used for direct manual annotation of gene products. It was created to be used for cross-referencing by other ontologies. Direct annotations to this term may be amended during annotation QC.